{
  "gene_name": "Coiled-coil domain-containing protein 170",
  "term_label": "microtubule cytoskeleton organization",
  "term_id": "GO:0000226",
  "gene_symbol": "CCDC170",
  "gene": "UniProtKB:Q8IYT3"
}